{
  "term_id": "GO:0007368",
  "gene": "UniProtKB:Q8WXU2",
  "gene_name": "Dynein axonemal assembly factor 4",
  "gene_symbol": "DNAAF4",
  "term_label": "determination of left/right symmetry"
}